regulation of tube diameter, open tracheal system [GO:0035158] (biological process) Also known as: regulation of tracheal tube diameter, tracheal tube dilation, tracheal tube expansion Relationships: is a type of regulation of tube size, open tracheal system [GO:0035151]; is a type of regulation of tube diameter [GO:0035296] Definition: Ensuring that a tube in an open tracheal system is of the correct diameter. When primary branches form their lumens are small (less than 2 micrometers) in caliber and must undergo regulated expansion during larval life to reach their mature size. References: PMID:14570584 Sources: GOC:mtg_sensu